{
  "gene": "UniProtKB:Q15596",
  "gene_symbol": "NCOA2",
  "term_id": "GO:0032870",
  "term_label": "cellular response to hormone stimulus",
  "gene_name": "Nuclear receptor coactivator 2"
}